{
  "gene_symbol": "CHD8",
  "gene_name": "Chromodomain-helicase-DNA-binding protein 8",
  "term_label": "ATP-dependent chromatin remodeler activity",
  "term_id": "GO:0140658",
  "gene": "UniProtKB:Q9HCK8"
}